{
  "gene_symbol": "PPP1R1C",
  "term_label": "intracellular signal transduction",
  "term_id": "GO:0035556",
  "gene": "UniProtKB:Q8WVI7",
  "gene_name": "Protein phosphatase 1 regulatory subunit 1C"
}